{
  "gene_symbol": "FAM43A",
  "gene_name": "Protein FAM43A",
  "gene": "UniProtKB:Q8N2R8",
  "term_label": "Unknown biological process",
  "term_id": "UNKNOWN:0002"
}